positive regulation of response to G1 DNA damage checkpoint signaling [GO:1902156] (biological process) Definition: Any process that activates or increases the frequency, rate or extent of response to G1 DNA damage checkpoint signaling. Relationships: is a type of positive regulation of response to DNA damage checkpoint signaling [GO:1902154]; is a type of regulation of response to G1 DNA damage checkpoint signaling [GO:1902155]; positively regulates response to G1 DNA damage checkpoint signaling [GO:0072432] Sources: GOC:TermGenie, GOC:mtg_cell_cycle Also known as: activation of mitotic cell cycle G1/S transition DNA damage checkpoint effector process, activation of response to mitotic cell cycle G1/S transition DNA damage checkpoint signaling, activation of response to signal involved in mitotic cell cycle G1/S transition DNA damage checkpoint, positive regulation of mitotic cell cycle G1/S transition DNA damage checkpoint effector process, positive regulation of response to mitotic cell cycle G1/S transition DNA damage checkpoint signaling, positive regulation of response to signal involved in mitotic cell cycle G1/S transition DNA damage checkpoint, up regulation of mitotic cell cycle G1/S transition DNA damage checkpoint effector process, up regulation of response to G1 DNA damage checkpoint signaling, up regulation of response to mitotic cell cycle G1/S transition DNA damage checkpoint signaling, up regulation of response to signal involved in mitotic cell cycle G1/S transition DNA damage checkpoint, up-regulation of mitotic cell cycle G1/S transition DNA damage checkpoint effector process, up-regulation of response to G1 DNA damage checkpoint signaling, up-regulation of response to mitotic cell cycle G1/S transition DNA damage checkpoint signaling, up-regulation of response to signal involved in mitotic cell cycle G1/S transition DNA damage checkpoint, upregulation of mitotic cell cycle G1/S transition DNA damage checkpoint effector process, upregulation of response to G1 DNA damage checkpoint signaling, upregulation of response to mitotic cell cycle G1/S transition DNA damage checkpoint signaling, upregulation of response to signal involved in mitotic cell cycle G1/S transition DNA damage checkpoint, activation of response to G1 DNA damage checkpoint signaling